tau protein binding [GO:0048156] (MF) Sources: GOC:jid Relationships: is a type of cytoskeletal protein binding [GO:0008092] Definition: Binding to tau protein. tau is a microtubule-associated protein, implicated in Alzheimer's disease, Down Syndrome and ALS.